3'-phosphoadenosine 5'-phosphosulfate binding [GO:0050656] (molecular function) Definition: Binding to 3'-phosphoadenosine 5'-phosphosulfate (PAPS), a naturally occurring mixed anhydride. It is an intermediate in the formation of a variety of sulfo compounds in biological systems. Sources: GOC:ai Also known as: 3'-phosphoadenosine 5'-phosphosulphate binding, 3'-phosphoadenylyl-sulfate binding, PAPS binding, adenosine 3'-phosphate 5'-phosphosulfate binding, phosphoadenosine phosphosulfate binding Relationships: is a type of adenyl ribonucleotide binding [GO:0032559]; is a type of GO:0043168; is a type of sulfur compound binding [GO:1901681]